{
  "gene_name": "Intracellular hyaluronan-binding protein 4",
  "term_label": "RNA binding",
  "gene_symbol": "HABP4",
  "gene": "UniProtKB:Q5JVS0",
  "term_id": "GO:0003723"
}